{
  "term_label": "protein monoubiquitination",
  "gene": "UniProtKB:Q9NS91",
  "gene_name": "E3 ubiquitin-protein ligase RAD18",
  "gene_symbol": "RAD18",
  "term_id": "GO:0006513"
}